{
  "gene_symbol": "ZNF99",
  "term_id": "GO:0005634",
  "gene": "UniProtKB:A8MXY4",
  "term_label": "nucleus",
  "gene_name": "Zinc finger protein 99"
}